regulation of defense response to oomycetes [GO:1902288] (biological process) Definition: Any process that modulates the frequency, rate or extent of defense response to oomycetes. Relationships: is a type of regulation of response to biotic stimulus [GO:0002831]; is a type of regulation of defense response [GO:0031347]; is a type of regulation of response to external stimulus [GO:0032101]; regulates defense response to oomycetes [GO:0002229] Subtypes: negative regulation of defense response to oomycetes [GO:1902289], GO:1902290 References: PMID:16040633 Sources: GOC:TermGenie